negative regulation of calcium ion export across plasma membrane [GO:1905913] (biological process) Definition: Any process that stops, prevents or reduces the frequency, rate or extent of calcium ion export across the plasma membrane. References: PMID:22362515 Sources: GOC:BHF, GOC:BHF_miRNA, GOC:TermGenie, GOC:rph, GO_REF:0000058 Also known as: down regulation of calcium ion efflux from cell, down regulation of calcium ion export from cell, down-regulation of calcium ion efflux from cell, down-regulation of calcium ion export from cell, downregulation of calcium ion efflux from cell, downregulation of calcium ion export from cell, negative regulation of calcium ion efflux from cell, negative regulation of calcium ion export from cell, inhibition of calcium ion efflux from cell, inhibition of calcium ion export from cell Relationships: is a type of negative regulation of calcium ion transmembrane transport [GO:1903170]; is a type of regulation of calcium ion export across plasma membrane [GO:1905912]; negatively regulates calcium ion export across plasma membrane [GO:1990034]